{
  "term_id": "GO:0006624",
  "gene_name": "Legumain",
  "gene_symbol": "LGMN",
  "term_label": "vacuolar protein processing",
  "gene": "UniProtKB:Q99538"
}